{
  "gene_symbol": "NME4",
  "term_label": "nucleoside diphosphate kinase activity",
  "gene": "UniProtKB:O00746",
  "gene_name": "Nucleoside diphosphate kinase, mitochondrial",
  "term_id": "GO:0004550"
}